flavonoid transport from endoplasmic reticulum to plant-type vacuole [GO:1903415] (biological process) Definition: The directed movement of flavonoid from endoplasmic reticulum to plant-type vacuole. References: PMID:25116949 Sources: GOC:TermGenie, GOC:tb, GO_REF:0000078 Also known as: flavonoid accumulation in vacuole Relationships: is a type of transport [GO:0006810]